{
  "term_id": "GO:0009986",
  "term_label": "cell surface",
  "gene_name": "Integrin beta-4",
  "gene": "UniProtKB:P16144",
  "gene_symbol": "ITGB4"
}